{
  "gene_symbol": "NCF1C",
  "gene": "UniProtKB:A8MVU1",
  "term_id": "GO:0043020",
  "term_label": "NADPH oxidase complex",
  "gene_name": "Putative neutrophil cytosol factor 1C"
}